{
  "gene_symbol": "CASP6",
  "term_label": "cysteine-type endopeptidase activity",
  "gene_name": "Caspase-6",
  "term_id": "GO:0004197",
  "gene": "UniProtKB:P55212"
}